{
  "gene": "UniProtKB:P0C7X3",
  "gene_symbol": "CCNYL3",
  "term_id": "GO:0005886",
  "term_label": "plasma membrane",
  "gene_name": "Putative cyclin-Y-like protein 3"
}